GABA-A receptor complex [GO:1902711] (cellular component) Note: An example of this is GBRA1 in human (UniProt symbol P14867) in PMID:18790874. Relationships: is a type of GO:1902710 Definition: A protein complex which is capable of GABA-A receptor activity. In human, it is usually composed of either two alpha, two beta and one gamma chain of the GABA-A receptor subunits or 5 chains of the GABA-A receptor subunits rho1-3 (formally known as GABA-C receptor). References: PMID:18790874 Sources: GOC:TermGenie, GOC:bhm, GO_REF:0000088